pronuclear envelope synthesis [GO:0018985] (biological process) Relationships: is a type of GO:0006998; is part of single fertilization [GO:0007338] Sources: GOC:ems Definition: Synthesis and ordering of the envelope of pronuclei. Subtypes: male pronuclear envelope synthesis [GO:0035043]